bleb assembly [GO:0032060] (biological process) Also known as: blebbing, membrane blebbing, cell blebbing, plasma membrane bleb assembly, plasma membrane blebbing Regulation: regulated by GO:1904170; negatively regulated by GO:1904171; positively regulated by positive regulation of bleb assembly [GO:1904172] References: PMID:12083798, PMID:16624291 Sources: GOC:mah, GOC:mtg_apoptosis, Wikipedia:Bleb_(cell_biology) Definition: The assembly of a bleb, a cell extension caused by localized decoupling of the cytoskeleton from the plasma membrane and characterized by rapid formation, rounded shape, and scarcity of organelles within the protrusion. Plasma membrane blebbing occurs during apoptosis and other cellular processes, including cell locomotion, cell division, and as a result of physical or chemical stresses. Relationships: is a type of GO:0120031